{
  "gene_name": "Grainyhead-like protein 1 homolog",
  "term_id": "GO:0001228",
  "gene_symbol": "GRHL1",
  "term_label": "DNA-binding transcription activator activity, RNA polymerase II-specific",
  "gene": "UniProtKB:Q9NZI5"
}